{
  "term_id": "GO:0043005",
  "gene_name": "Fragile X messenger ribonucleoprotein 1",
  "gene_symbol": "FMR1",
  "term_label": "neuron projection",
  "gene": "UniProtKB:Q06787"
}